{
  "term_id": "GO:0000977",
  "term_label": "RNA polymerase II transcription regulatory region sequence-specific DNA binding",
  "gene_symbol": "ZNF599",
  "gene": "UniProtKB:Q96NL3",
  "gene_name": "Zinc finger protein 599"
}